{
  "term_label": "cell surface receptor signaling pathway",
  "gene": "UniProtKB:A0A539",
  "gene_name": "T cell receptor beta variable 4-2",
  "gene_symbol": "TRBV4-2",
  "term_id": "GO:0007166"
}